{
  "term_id": "UNKNOWN:0003",
  "gene_name": "Endosomal transmembrane epsin interactor 1",
  "gene_symbol": "ENTREP1",
  "term_label": "Unknown cellular component",
  "gene": "UniProtKB:Q15884"
}